positive regulation of gamma-aminobutyric acid catabolic process [GO:1901717] (biological process) Also known as: activation of 4-aminobutanoate catabolic process, activation of 4-aminobutanoate catabolism, activation of 4-aminobutyrate catabolic process, activation of 4-aminobutyrate catabolism, activation of GABA catabolic process, activation of GABA catabolism, activation of gamma-aminobutyric acid breakdown, activation of gamma-aminobutyric acid catabolism, activation of gamma-aminobutyric acid degradation, positive regulation of 4-aminobutanoate catabolic process, positive regulation of 4-aminobutanoate catabolism, positive regulation of 4-aminobutyrate catabolic process, positive regulation of 4-aminobutyrate catabolism, positive regulation of GABA catabolic process, positive regulation of GABA catabolism, positive regulation of gamma-aminobutyric acid breakdown, positive regulation of gamma-aminobutyric acid catabolism, positive regulation of gamma-aminobutyric acid degradation, up regulation of 4-aminobutanoate catabolic process, up regulation of 4-aminobutanoate catabolism, up regulation of 4-aminobutyrate catabolic process, up regulation of 4-aminobutyrate catabolism, up regulation of GABA catabolic process, up regulation of GABA catabolism, up regulation of gamma-aminobutyric acid breakdown, up regulation of gamma-aminobutyric acid catabolic process, up regulation of gamma-aminobutyric acid catabolism, up regulation of gamma-aminobutyric acid degradation, up-regulation of 4-aminobutanoate catabolic process, up-regulation of 4-aminobutanoate catabolism, up-regulation of 4-aminobutyrate catabolic process, up-regulation of 4-aminobutyrate catabolism, up-regulation of GABA catabolic process, up-regulation of GABA catabolism, up-regulation of gamma-aminobutyric acid breakdown, up-regulation of gamma-aminobutyric acid catabolic process, up-regulation of gamma-aminobutyric acid catabolism, up-regulation of gamma-aminobutyric acid degradation, upregulation of 4-aminobutanoate catabolic process, upregulation of 4-aminobutanoate catabolism, upregulation of 4-aminobutyrate catabolic process, upregulation of 4-aminobutyrate catabolism, upregulation of GABA catabolic process, upregulation of GABA catabolism, upregulation of gamma-aminobutyric acid breakdown, upregulation of gamma-aminobutyric acid catabolic process, upregulation of gamma-aminobutyric acid catabolism, upregulation of gamma-aminobutyric acid degradation, activation of gamma-aminobutyric acid catabolic process Relationships: is a type of GO:0009896; is a type of positive regulation of amino acid metabolic process [GO:0045764]; is a type of GO:0062013; is a type of GO:1901715; positively regulates GO:0009450 Definition: Any process that activates or increases the frequency, rate or extent of gamma-aminobutyric acid catabolic process. Sources: GOC:TermGenie